{
  "gene": "UniProtKB:Q96NI6",
  "term_label": "Unknown molecular function",
  "term_id": "UNKNOWN:0001",
  "gene_symbol": "LRFN5",
  "gene_name": "Leucine-rich repeat and fibronectin type-III domain-containing protein 5"
}